chlorophyll binding [GO:0016168] (molecular function) Definition: Binding to a chlorophyll; a compound of magnesium complexed in a porphyrin (tetrapyrrole) ring and which functions as a photosynthetic pigment. Relationships: is_a tetrapyrrole binding [GO:0046906] Sources: GOC:jl Subtypes: bacteriochlorophyll binding [GO:0042314]